synaptic membrane adhesion to extracellular matrix [GO:0099561] (BP) Sources: GOC:dos Definition: The binding of a synaptic membrane to the extracellular matrix via adhesion molecules. Relationships: is a type of GO:0007160; is part of synapse organization [GO:0050808]